{
  "term_label": "inflammatory response",
  "gene_symbol": "TLR4",
  "term_id": "GO:0006954",
  "gene": "UniProtKB:O00206",
  "gene_name": "Toll-like receptor 4"
}